{
  "gene_name": "Transcription elongation factor A protein-like 7",
  "gene_symbol": "TCEAL7",
  "term_id": "UNKNOWN:0002",
  "gene": "UniProtKB:Q9BRU2",
  "term_label": "Unknown biological process"
}